{
  "gene_symbol": "KLHL10",
  "term_id": "GO:0031463",
  "gene_name": "Kelch-like protein 10",
  "term_label": "Cul3-RING ubiquitin ligase complex",
  "gene": "UniProtKB:Q6JEL2"
}